{
  "term_label": "Unknown cellular component",
  "gene_name": "TBC1 domain family member 10B",
  "term_id": "UNKNOWN:0003",
  "gene": "UniProtKB:Q4KMP7",
  "gene_symbol": "TBC1D10B"
}